{
  "gene_symbol": "H1-0",
  "term_id": "GO:0045910",
  "gene": "UniProtKB:P07305",
  "gene_name": "Histone H1.0",
  "term_label": "negative regulation of DNA recombination"
}